dense core granule maturation [GO:1990502] (biological process) Definition: Steps required to transform a dense core granule generated at the trans-Golgi network into a fully formed and transmissible dense core granule. Dense core granule maturation proceeds through clathrin-mediated membrane remodeling events and is essential for efficient processing of cargo within dense core granules as well as for removing factors that might otherwise interfere with dense core granule trafficking and exocytosis. References: PMID:22654674 Sources: GOC:kmv Also known as: dense core vesicle maturation Relationships: is_a secretory granule maturation [GO:0061792]